{
  "gene_symbol": "KIF5C",
  "term_label": "kinesin complex",
  "gene_name": "Kinesin heavy chain isoform 5C",
  "term_id": "GO:0005871",
  "gene": "UniProtKB:O60282"
}